chlorophyll a catabolic process [GO:0033310] (biological process) Sources: GOC:mah Relationships: is a type of chlorophyll catabolic process [GO:0015996] Definition: The chemical reactions and pathways leading to the breakdown of chlorophyll a. Also known as: chlorophyll a breakdown, chlorophyll a catabolism, chlorophyll a degradation